{
  "gene": "UniProtKB:Q9H1H9",
  "term_id": "GO:0007018",
  "gene_symbol": "KIF13A",
  "term_label": "microtubule-based movement",
  "gene_name": "Kinesin-like protein KIF13A"
}